{
  "gene": "UniProtKB:Q5SYC1",
  "gene_symbol": "CLVS2",
  "term_id": "GO:0005802",
  "term_label": "trans-Golgi network",
  "gene_name": "Clavesin-2"
}